{
  "term_id": "UNKNOWN:0003",
  "gene_symbol": "RAB36",
  "gene": "UniProtKB:O95755",
  "term_label": "Unknown cellular component",
  "gene_name": "Ras-related protein Rab-36"
}